{
  "term_id": "GO:0006307",
  "gene_symbol": "ALKBH2",
  "gene": "UniProtKB:Q6NS38",
  "term_label": "DNA alkylation repair",
  "gene_name": "DNA oxidative demethylase ALKBH2"
}